{
  "term_label": "regulation of cytokinesis",
  "term_id": "GO:0032465",
  "gene_name": "Rab11 family-interacting protein 3",
  "gene_symbol": "RAB11FIP3",
  "gene": "UniProtKB:O75154"
}